{
  "gene_name": "G2_mitotic-specific cyclin-B1",
  "gene": "UniProtKB:P14635",
  "term_label": "cyclin-dependent protein serine/threonine kinase regulator activity",
  "term_id": "GO:0016538",
  "gene_symbol": "CCNB1"
}